{
  "gene_name": "High mobility group protein 20A",
  "term_label": "regulation of gene expression",
  "term_id": "GO:0010468",
  "gene": "UniProtKB:Q9NP66",
  "gene_symbol": "HMG20A"
}